formylmethanofuran-tetrahydromethanopterin N-formyltransferase activity [GO:0030270] (molecular function) Also known as: FTR, N-formylmethanofuran(CHO-MFR):tetrahydromethanopterin(H4MPT) formyltransferase activity, formylmethanofuran-tetrahydromethanopterin formyltransferase activity, formylmethanofuran:5,6,7,8-tetrahydromethanopterin 5-formyltransferase activity, formylmethanofuran:5,6,7,8-tetrahydromethanopterin N5-formyltransferase activity, formylmethanofuran:tetrahydromethanopterin formyltransferase activity Definition: Catalysis of the reaction: 5,6,7,8-tetrahydromethanopterin + N-formylmethanofuran + H+ = N(5)-formyl-5,6,7,8-tetrahydromethanopterin + methanofuran. Sources: EC:2.3.1.101, RHEA:18061 Relationships: is_a N-acyltransferase activity [GO:0016410]